{
  "gene_name": "Cytokine SCM-1 beta",
  "gene_symbol": "XCL2",
  "term_id": "GO:0061844",
  "term_label": "antimicrobial humoral immune response mediated by antimicrobial peptide",
  "gene": "UniProtKB:Q9UBD3"
}